{
  "term_id": "UNKNOWN:0001",
  "gene_symbol": "RBM43",
  "gene": "UniProtKB:Q6ZSC3",
  "gene_name": "RNA-binding protein 43",
  "term_label": "Unknown molecular function"
}